negative regulation of myeloid leukocyte mediated immunity [GO:0002887] (biological process) Also known as: down regulation of myeloid leukocyte mediated immunity, down-regulation of myeloid leukocyte mediated immunity, downregulation of myeloid leukocyte mediated immunity, inhibition of myeloid leukocyte mediated immunity Relationships: is a type of negative regulation of leukocyte mediated immunity [GO:0002704]; is a type of regulation of myeloid leukocyte mediated immunity [GO:0002886]; negatively regulates myeloid leukocyte mediated immunity [GO:0002444] Subtypes: negative regulation of type III hypersensitivity [GO:0001804], negative regulation of myeloid dendritic cell cytokine production [GO:0002734], negative regulation of type II hypersensitivity [GO:0002893], negative regulation of mast cell degranulation [GO:0043305], negative regulation of eosinophil degranulation [GO:0043310], GO:0043314, GO:0070954, GO:1903582, GO:1904150 Sources: GOC:add Definition: Any process that stops, prevents, or reduces the frequency, rate, or extent of myeloid leukocyte mediated immunity.